regulation of response to tumor cell [GO:0002834] (biological process) Definition: Any process that modulates the frequency, rate, or extent of a response to tumor cell. Sources: GOC:add Also known as: regulation of response to tumour cell Relationships: is a type of regulation of response to biotic stimulus [GO:0002831]; regulates response to tumor cell [GO:0002347] Subtypes: GO:0002835, positive regulation of response to tumor cell [GO:0002836], GO:0002837